{
  "term_label": "actin filament bundle assembly",
  "gene": "UniProtKB:Q9BQI0",
  "gene_name": "Allograft inflammatory factor 1-like",
  "gene_symbol": "AIF1L",
  "term_id": "GO:0051017"
}